{
  "gene": "UniProtKB:Q8WVV4",
  "gene_symbol": "POF1B",
  "term_id": "GO:0003382",
  "term_label": "epithelial cell morphogenesis",
  "gene_name": "Protein POF1B"
}